{
  "gene": "UniProtKB:Q5VW36",
  "term_label": "Unknown biological process",
  "gene_symbol": "FOCAD",
  "term_id": "UNKNOWN:0002",
  "gene_name": "Focadhesin"
}